positive regulation of ATF6-mediated unfolded protein response [GO:1903893] (biological process) References: PMID:22013210 Sources: GOC:PARL, GOC:TermGenie, GOC:bf, GO_REF:0000058 Relationships: is a type of positive regulation of endoplasmic reticulum unfolded protein response [GO:1900103]; is a type of regulation of ATF6-mediated unfolded protein response [GO:1903891]; positively regulates ATF6-mediated unfolded protein response [GO:0036500] Definition: Any process that activates or increases the frequency, rate or extent of the ATF6-mediated unfolded protein response. Also known as: positive regulation of ATF6 branch of UPR, positive regulation of UPR signaling by ATF6 stress sensor, positive regulation of activating transcription factor 6 signaling in unfolded protein response, positive regulation of endoplasmic reticulum unfolded protein response; ATF6 signaling, up regulation of ATF6 branch of UPR, up regulation of ATF6-mediated unfolded protein response, up regulation of UPR signaling by ATF6 stress sensor, up regulation of activating transcription factor 6 signaling in unfolded protein response, up regulation of endoplasmic reticulum unfolded protein response; ATF6 signaling, up-regulation of ATF6 branch of UPR, up-regulation of ATF6-mediated unfolded protein response, up-regulation of UPR signaling by ATF6 stress sensor, up-regulation of activating transcription factor 6 signaling in unfolded protein response, up-regulation of endoplasmic reticulum unfolded protein response; ATF6 signaling, upregulation of ATF6 branch of UPR, upregulation of ATF6-mediated unfolded protein response, upregulation of UPR signaling by ATF6 stress sensor, upregulation of activating transcription factor 6 signaling in unfolded protein response, upregulation of endoplasmic reticulum unfolded protein response; ATF6 signaling, activation of ATF6 branch of UPR, activation of ATF6-alpha UPR branch, activation of ATF6-beta UPR branch, activation of ATF6-mediated unfolded protein response, activation of UPR signaling by ATF6 stress sensor, activation of activating transcription factor 6 signaling in unfolded protein response, activation of endoplasmic reticulum unfolded protein response; ATF6 signaling, positive regulation of ATF6-alpha UPR branch, positive regulation of ATF6-beta UPR branch, up regulation of ATF6-alpha UPR branch, up regulation of ATF6-beta UPR branch, up-regulation of ATF6-alpha UPR branch, up-regulation of ATF6-beta UPR branch, upregulation of ATF6-alpha UPR branch, upregulation of ATF6-beta UPR branch, activation of ATF6 signaling in response to endoplasmic reticulum stress, positive regulation of ATF6 signaling in response to endoplasmic reticulum stress, up regulation of ATF6 signaling in response to endoplasmic reticulum stress, up-regulation of ATF6 signaling in response to endoplasmic reticulum stress, upregulation of ATF6 signaling in response to endoplasmic reticulum stress